neurotransmitter transmembrane transporter activity [GO:0005326] (molecular function) Definition: Enables the directed movement of a neurotransmitter into, out of or within a cell, or between cells. Neurotransmitters are any chemical substance that is capable of transmitting (or inhibiting the transmission of) a nerve impulse from a neuron to another cell. Sources: GOC:ai, ISBN:0198506732 Also known as: neurotransmitter transporter activity Relationships: is a type of transmembrane transporter activity [GO:0022857]; is part of neurotransmitter transport [GO:0006836] Subtypes: acetylcholine transmembrane transporter activity [GO:0005277], neurotransmitter:sodium symporter activity [GO:0005328]